{
  "term_label": "Unknown biological process",
  "term_id": "UNKNOWN:0002",
  "gene": "UniProtKB:A2A2V5",
  "gene_name": "Serine-rich and transmembrane domain-containing protein 1",
  "gene_symbol": "SERTM1"
}